{
  "gene_symbol": "SOX18",
  "term_label": "DNA-binding transcription activator activity, RNA polymerase II-specific",
  "gene": "UniProtKB:P35713",
  "gene_name": "Transcription factor SOX-18",
  "term_id": "GO:0001228"
}